{
  "gene_name": "Leucine-rich alpha-2-glycoprotein",
  "term_label": "positive regulation of transforming growth factor beta receptor signaling pathway",
  "gene_symbol": "LRG1",
  "gene": "UniProtKB:P02750",
  "term_id": "GO:0030511"
}